negative regulation of juvenile hormone metabolic process [GO:0045928] (biological process) Sources: GOC:go_curators Also known as: down regulation of juvenile hormone metabolic process, down-regulation of juvenile hormone metabolic process, downregulation of juvenile hormone metabolic process, negative regulation of juvenile hormone metabolism, inhibition of juvenile hormone metabolic process Definition: Any process that stops, prevents, or reduces the frequency, rate or extent of the chemical reactions and pathways involving juvenile hormone. Relationships: is a type of negative regulation of hormone metabolic process [GO:0032351]; is a type of negative regulation of isoprenoid metabolic process [GO:0045827]; negatively regulates juvenile hormone metabolic process [GO:0006716] Subtypes: GO:0045968, negative regulation of juvenile hormone catabolic process [GO:0045970]